hydrolase activity, acting on carbon-nitrogen (but not peptide) bonds [GO:0016810] (molecular function) Also known as: hydrolase activity, acting on carbon-nitrogen (but not peptide) bonds, in other compounds Subtypes: GO:0009392, GO:0010178, hydrolase activity, acting on carbon-nitrogen (but not peptide) bonds, in linear amides [GO:0016811], hydrolase activity, acting on carbon-nitrogen (but not peptide) bonds, in cyclic amides [GO:0016812], hydrolase activity, acting on carbon-nitrogen (but not peptide) bonds, in linear amidines [GO:0016813], hydrolase activity, acting on carbon-nitrogen (but not peptide) bonds, in cyclic amidines [GO:0016814], hydrolase activity, acting on carbon-nitrogen (but not peptide) bonds, in nitriles [GO:0016815], strictosidine synthase activity [GO:0016844], hydroxydechloroatrazine ethylaminohydrolase activity [GO:0018763], N-isopropylammelide isopropylaminohydrolase activity [GO:0018764], deaminase activity [GO:0019239], riboflavinase activity [GO:0050258], thiaminase activity [GO:0050334], (S)-norcoclaurine synthase activity [GO:0050474], deacetylisoipecoside synthase activity [GO:0050556], deacetylipecoside synthase activity [GO:0050557], jasmonic acid hydrolase [GO:0120091], GO:1990206 Relationships: is a type of hydrolase activity [GO:0016787] Definition: Catalysis of the hydrolysis of any carbon-nitrogen bond, C-N, with the exception of peptide bonds. Sources: EC:3.5.-.-